{
  "term_label": "mitochondrial membrane",
  "term_id": "GO:0031966",
  "gene_symbol": "COX6C",
  "gene": "UniProtKB:P09669",
  "gene_name": "Cytochrome c oxidase subunit 6C"
}